{
  "term_id": "UNKNOWN:0003",
  "gene_name": "Uncharacterized protein",
  "gene": "UniProtKB:A0A8V8TNB9",
  "term_label": "Unknown cellular component",
  "gene_symbol": "A0A8V8TNB9"
}